{
  "term_label": "RNA polymerase II C-terminal domain phosphoserine binding",
  "gene": "UniProtKB:O95104",
  "gene_name": "SR-related and CTD-associated factor 4",
  "gene_symbol": "SCAF4",
  "term_id": "GO:1990269"
}